{
  "term_label": "metalloendopeptidase activity",
  "gene": "UniProtKB:O75078",
  "gene_name": "Disintegrin and metalloproteinase domain-containing protein 11",
  "term_id": "GO:0004222",
  "gene_symbol": "ADAM11"
}